{
  "term_label": "regulation of transcription by RNA polymerase II",
  "gene_symbol": "SCX",
  "gene": "UniProtKB:Q7RTU7",
  "term_id": "GO:0006357",
  "gene_name": "Basic helix-loop-helix transcription factor scleraxis"
}